{
  "term_label": "brush border",
  "gene": "UniProtKB:Q06495",
  "gene_name": "Sodium-dependent phosphate transport protein 2A",
  "term_id": "GO:0005903",
  "gene_symbol": "SLC34A1"
}